oligodendrocyte apoptotic process [GO:0097252] (biological process) Definition: Any apoptotic process in an oligodendrocyte. Oligodendrocytes belong to a class of large neuroglial (macroglial) cells in the central nervous system, where they form the insulating myelin sheath of axons. References: PMID:16723520 Sources: CL:0000128, GOC:mtg_apoptosis, GOC:yaf Also known as: oligodendrocyte apoptosis Relationships: is a type of glial cell apoptotic process [GO:0034349] Regulation: RO_0002211 by GO:1900141; negatively regulated by GO:1900142; positively regulated by GO:1900143